superior temporal gyrus development [GO:0071109] (BP) Definition: The process whose specific outcome is the progression of the superior temporal gyrus over time, from its formation to the mature structure. The superior temporal gyrus is a portion of the cerebral cortex that extends from the lateral sulcus to the superior temporal sulcus. References: PMID:11484000 Sources: FMA:61905, GOC:BHF, GOC:mah Relationships: is a type of GO:0048856; is part of cerebral cortex development [GO:0021987]